{
  "gene_name": "PR domain zinc finger protein 4",
  "gene": "UniProtKB:Q9UKN5",
  "gene_symbol": "PRDM4",
  "term_id": "GO:0000981",
  "term_label": "DNA-binding transcription factor activity, RNA polymerase II-specific"
}